{
  "gene_name": "Reactive oxygen species modulator 1",
  "gene_symbol": "ROMO1",
  "term_id": "GO:0030150",
  "gene": "UniProtKB:P60602",
  "term_label": "protein import into mitochondrial matrix"
}